{
  "gene": "UniProtKB:A6NJG2",
  "gene_name": "Ankyrin repeat domain-containing protein SOWAHD",
  "term_label": "Unknown cellular component",
  "term_id": "UNKNOWN:0003",
  "gene_symbol": "SOWAHD"
}